{
  "gene_symbol": "LINC01549",
  "term_id": "UNKNOWN:0001",
  "gene": "UniProtKB:A6NIU2",
  "term_label": "Unknown molecular function",
  "gene_name": "Putative uncharacterized protein encoded by LINC01549"
}